{
  "term_label": "entrainment of circadian clock by photoperiod",
  "term_id": "GO:0043153",
  "gene_symbol": "PER2",
  "gene": "UniProtKB:O15055",
  "gene_name": "Period circadian protein homolog 2"
}